polyprenyldihydroxybenzoate methyltransferase activity [GO:0010420] (molecular function) References: PMID:10419476, PMID:23190198, PMID:9628017 Sources: RHEA:44452 Note: Note that the polyprenyl sidechain substrate for this reaction has a different number of prenyl units in different organisms (for example, ubiquinone-6 in Saccharomyces, ubiquinone- 9 in rat and ubiquinone-10 in human), and thus the natural substrate for the enzymes from different organisms has a different number of prenyl units. However, the enzyme usually shows a low degree of specificity regarding the number of prenyl units. Definition: Catalysis of the reaction: a 3,4-dihydroxy-5-all-trans-polyprenylbenzoate + S-adenosyl-L-methionine = a 3-methoxy,4-hydroxy-5-all-trans-polyprenylbenzoate + S-adenosyl-L-homocysteine + H+. Also known as: 3,4-dihydroxy-5-polyprenylbenzoic acid O-methyltransferase activity Relationships: is a type of S-adenosylmethionine-dependent methyltransferase activity [GO:0008757]; is part of ubiquinone biosynthetic process [GO:0006744]